macrolide transmembrane transporter complex [GO:1990195] (cellular component) Definition: A bacterial transmembrane transporter complex that spans the entire cell membrane system and possesses ATP-dependent xenobiotic transport activity pumping drugs (typically antibiotics) and other toxins directly from the cytosol out of the bacterial cell. Typically, it is trimeric consisting of a inner membrane ATPase (IMP), a periplasmic membrane fusion protein (MFP) and an outer membrane factor (OMF). In E. coli, macrolide transporter complexes may consists of MacB (IMP), MacA (MFP) and TolC (OMF) or AcrB (IMP), AcrA (MFP) and TolC (OMF). Trimeric TolC is a common OMF found in many macrolide transporter complexes. References: PMID:10879525, PMID:18955484, PMID:19254725 Sources: GOC:bhm Also known as: macrolide transporter complex, AcrAB-TolC complex, MacAB-TolC complex, macrolide transporter Relationships: is a type of transmembrane transporter complex [GO:1902495] Subtypes: MacAB-TolC complex [GO:1990196]